{
  "term_label": "Unknown molecular function",
  "gene": "UniProtKB:Q8N9T8",
  "term_id": "UNKNOWN:0001",
  "gene_name": "Protein KRI1 homolog",
  "gene_symbol": "KRI1"
}